{
  "term_label": "omega-amidase activity",
  "gene": "UniProtKB:Q9NQR4",
  "term_id": "GO:0050152",
  "gene_symbol": "NIT2",
  "gene_name": "Omega-amidase NIT2"
}